{
  "gene": "UniProtKB:O00221",
  "gene_symbol": "NFKBIE",
  "term_label": "protein sequestering activity",
  "term_id": "GO:0140311",
  "gene_name": "NF-kappa-B inhibitor epsilon"
}